negative regulation of transcription initiation by RNA polymerase II [GO:0060633] (biological process) Definition: Any process that decreases the rate, frequency or extent of a process involved in starting transcription from an RNA polymerase II promoter. Sources: GOC:dph, GOC:tb, GOC:txnOH Also known as: negative regulation of transcription initiation from RNA polymerase II promoter Relationships: is a type of negative regulation of transcription by RNA polymerase II [GO:0000122]; is a type of regulation of transcription initiation by RNA polymerase II [GO:0060260]; is_a negative regulation of DNA-templated transcription initiation [GO:2000143]; negatively regulates transcription initiation at RNA polymerase II promoter [GO:0006367] Subtypes: GO:0017055